NAD+ nucleosidase activity [GO:0003953] (molecular function) Definition: Catalysis of the reaction: NAD+ + H2O = ADP-D-ribose + nicotinamide + H+. References: PMID:11866528, PMID:7805847 Sources: RHEA:16301 Also known as: DPNase activity, NAD glycohydrolase activity, NAD nucleosidase activity, NAD(+) glycohydrolase activity, NADase activity, beta-NAD(+) glycohydrolase activity, diphosphopyridine nucleosidase activity, nicotinamide adenine dinucleotide glycohydrolase activity, nicotinamide adenine dinucleotide nucleosidase activity Relationships: is a type of hydrolase activity, hydrolyzing N-glycosyl compounds [GO:0016799]